{
  "gene_name": "Olfactory receptor 4N2",
  "gene": "UniProtKB:Q8NGD1",
  "term_label": "olfactory receptor activity",
  "gene_symbol": "OR4N2",
  "term_id": "GO:0004984"
}